{
  "term_label": "regulation of dendritic spine morphogenesis",
  "term_id": "GO:0061001",
  "gene": "UniProtKB:O14559",
  "gene_name": "Rho GTPase-activating protein 33",
  "gene_symbol": "ARHGAP33"
}